{
  "gene_name": "Cbp_p300-interacting transactivator 4",
  "gene": "UniProtKB:Q96RK1",
  "gene_symbol": "CITED4",
  "term_label": "nucleus",
  "term_id": "GO:0005634"
}